symbiont-mediated suppression of host cytoplasmic pattern recognition receptor signaling pathway via inhibition of MAVS activity [GO:0039545] (biological process) Definition: A process in which a symbiont interferes with, inhibits or disrupts a cytoplasmic pattern recognition receptor signaling pathway in a host organism by reducing the activity of host MAVS (mitochondrial antiviral signaling protein). MAVS is a signal transducer that lies downstream of the viral RNA receptors MDA-5 and RIG-I to coordinate host innate immune responses. References: PMID:17438296, PMID:22674996 Also known as: suppression by virus of host viral-induced cytoplasmic pattern recognition receptor signaling pathway via inhibition of MAVS activity, inhibition of host MAVS by virus, suppression by virus of host MAVS activity, suppression by virus of host mitochondrial antiviral-signaling protein Note: This term is for annotation of symbiont proteins that counteract the host anti-microbial innate immune response. Relationships: is a type of GO:0039537